{
  "gene": "UniProtKB:Q14593",
  "gene_name": "Zinc finger protein 273",
  "term_id": "GO:0000981",
  "gene_symbol": "ZNF273",
  "term_label": "DNA-binding transcription factor activity, RNA polymerase II-specific"
}